{
  "gene_name": "Uncharacterized protein FLJ37310",
  "gene_symbol": "Q8N1X5",
  "term_id": "UNKNOWN:0001",
  "term_label": "Unknown molecular function",
  "gene": "UniProtKB:Q8N1X5"
}